{
  "gene_symbol": "ADAMTS8",
  "term_label": "proteolysis",
  "gene_name": "A disintegrin and metalloproteinase with thrombospondin motifs 8",
  "term_id": "GO:0006508",
  "gene": "UniProtKB:Q9UP79"
}